{
  "term_id": "UNKNOWN:0001",
  "gene": "UniProtKB:A6NGS2",
  "gene_symbol": "ERICH4",
  "term_label": "Unknown molecular function",
  "gene_name": "Glutamate-rich protein 4"
}